{
  "gene_name": "Transmembrane protein 26",
  "gene": "UniProtKB:Q6ZUK4",
  "term_id": "UNKNOWN:0001",
  "term_label": "Unknown molecular function",
  "gene_symbol": "TMEM26"
}